{
  "term_id": "GO:0004622",
  "gene_name": "Lysophospholipase D GDPD1",
  "gene_symbol": "GDPD1",
  "term_label": "phosphatidylcholine lysophospholipase activity",
  "gene": "UniProtKB:Q8N9F7"
}